{
  "term_label": "nucleus",
  "gene_name": "Pantothenate kinase 1",
  "term_id": "GO:0005634",
  "gene": "UniProtKB:Q8TE04",
  "gene_symbol": "PANK1"
}